nuclear polyadenylation-dependent ncRNA catabolic process [GO:0071046] (biological process) Relationships: is a type of nuclear RNA surveillance [GO:0071027] Also known as: nuclear poly(A)-dependent ncRNA catabolic process Definition: The chemical reactions and pathways occurring in the nucleus and resulting in the breakdown of a noncoding RNA (ncRNA) molecule, initiated by the enzymatic addition of a sequence of adenylyl residues (polyadenylation) at the 3' end the target ncRNA. References: PMID:17410208 Sources: GOC:dgf, GOC:jl, GOC:krc